surfactant homeostasis [GO:0043129] (biological process) Definition: Any process involved in the maintenance of a steady-state level of a surface-active agent that maintains the surface tension of a liquid. References: PMID:23708874, PMID:9751757 Also known as: regulation of liquid surface tension, regulation of surface tension of a liquid, surfactant activity Relationships: is a type of multicellular organismal-level chemical homeostasis [GO:0140962]